{
  "term_label": "negative regulation of transcription by RNA polymerase II",
  "gene_name": "Zinc finger protein 782",
  "gene_symbol": "ZNF782",
  "gene": "UniProtKB:Q6ZMW2",
  "term_id": "GO:0000122"
}